{
  "term_label": "humoral immune response",
  "term_id": "GO:0006959",
  "gene": "UniProtKB:P01570",
  "gene_name": "Interferon alpha-14",
  "gene_symbol": "IFNA14"
}